{
  "term_label": "Unknown cellular component",
  "gene_symbol": "JOSD2",
  "gene_name": "Josephin-2",
  "term_id": "UNKNOWN:0003",
  "gene": "UniProtKB:Q8TAC2"
}